{
  "gene_name": "AP-1 complex subunit gamma-like 2",
  "gene_symbol": "AP1G2",
  "term_label": "AP-1 adaptor complex",
  "gene": "UniProtKB:O75843",
  "term_id": "GO:0030121"
}